mesonephric juxtaglomerulus cell differentiation [GO:0061207] (BP) Definition: The process in which relatively unspecialized cells acquire specialized structural and/or functional features that characterize the juxtaglomerulus cells of the mesonephros as it progresses from its formation to the mature state. Relationships: is a type of GO:0061208; is a type of juxtaglomerulus cell differentiation [GO:0072052]; is part of mesonephric juxtaglomerular apparatus development [GO:0061212] Sources: GOC:mtg_kidney_jan10